{
  "term_label": "Unknown biological process",
  "gene_symbol": "CCDC50",
  "gene": "UniProtKB:Q8IVM0",
  "term_id": "UNKNOWN:0002",
  "gene_name": "Coiled-coil domain-containing protein 50"
}